dimethylallylcistransferase activity [GO:0047863] (molecular function) Also known as: dimethylallyl-diphosphate:isopentenyl-diphosphate dimethylallylcistransferase activity, neryl-diphosphate synthase activity Sources: RHEA:11328 Relationships: is a type of prenyl diphosphate synthase activity [GO:0120531] Definition: Catalysis of the reaction: dimethylallyl diphosphate + isopentenyl diphosphate = diphosphate + neryl diphosphate.